{
  "gene": "UniProtKB:Q99967",
  "gene_symbol": "CITED2",
  "term_label": "sex determination",
  "gene_name": "Cbp_p300-interacting transactivator 2",
  "term_id": "GO:0007530"
}